{
  "term_label": "nucleus",
  "gene": "UniProtKB:Q9UBF1",
  "gene_symbol": "MAGEC2",
  "gene_name": "Melanoma-associated antigen C2",
  "term_id": "GO:0005634"
}